D-glucose transmembrane transporter activity [GO:0055056] (MF) Relationships: is a type of hexose transmembrane transporter activity [GO:0015149] Sources: GOC:jid, GOC:jsg, GOC:mah Definition: Enables the transfer of the D-enantiomer of the hexose monosaccharide glucose from one side of a membrane to the other. Subtypes: D-glucose:proton symporter activity [GO:0005356], D-glucose:sodium symporter activity [GO:0005412], D-glucose uniporter activity [GO:0015304], protein-N(PI)-phosphohistidine-glucose phosphotransferase system transporter activity [GO:0022855], protein-N(PI)-phosphohistidine-sorbose phosphotransferase system transporter activity [GO:0022871], GO:0022881, GO:0140108